mesonephric nephron morphogenesis [GO:0061228] (biological process) Sources: GOC:mtg_kidney_jan10 Definition: The process in which the anatomical structures of the mesonephric nephron are generated and organized. A mesonephric nephron is the functional unit of the mesonephros. Relationships: is a type of nephron morphogenesis [GO:0072028]; is part of GO:0061206; is part of mesonephric nephron development [GO:0061215]